medium-chain fatty aldehyde dehydrogenase (NAD+) activity [GO:0052814] (molecular function) Relationships: is a type of fatty aldehyde dehydrogenase (NAD+) activity [GO:0102673] Definition: Catalysis of the reaction: a medium-chain fatty aldehyde + H2O + NAD+ = a medium chain fatty acid + 2 H+ + NADH. Also known as: medium-chain-aldehyde dehydrogenase activity, medium-chain aliphatic aldehyde dehydrogenase activity, medium-chain fatty aldehyde dehydrogenase activity, medium-chain-aldehyde:NAD+ oxidoreductase activity Sources: RHEA:69763